epidermis development [GO:0008544] (biological process) Subtypes: skin epidermis development [GO:0098773] Regulation: regulated by regulation of epidermis development [GO:0045682]; negatively regulated by negative regulation of epidermis development [GO:0045683]; positively regulated by positive regulation of epidermis development [GO:0045684] Definition: The process whose specific outcome is the progression of the epidermis over time, from its formation to the mature structure. The epidermis is the outer epithelial layer of an animal, it may be a single layer that produces an extracellular material (e.g. the cuticle of arthropods) or a complex stratified squamous epithelium, as in the case of many vertebrate species. Also known as: hypodermis development Sources: GOC:go_curators, UBERON:0001003 Relationships: is a type of tissue development [GO:0009888]